{
  "gene": "UniProtKB:Q05209",
  "gene_name": "Tyrosine-protein phosphatase non-receptor type 12",
  "term_id": "GO:0004725",
  "term_label": "protein tyrosine phosphatase activity",
  "gene_symbol": "PTPN12"
}